{
  "term_id": "GO:0005737",
  "gene_symbol": "PPIC",
  "gene": "UniProtKB:P45877",
  "gene_name": "Peptidyl-prolyl cis-trans isomerase C",
  "term_label": "cytoplasm"
}